{
  "gene": "UniProtKB:Q8NFT2",
  "term_label": "copper ion import",
  "term_id": "GO:0015677",
  "gene_name": "Metalloreductase STEAP2",
  "gene_symbol": "STEAP2"
}